{
  "gene_name": "Maspardin",
  "gene_symbol": "SPG21",
  "term_id": "GO:0030140",
  "gene": "UniProtKB:Q9NZD8",
  "term_label": "trans-Golgi network transport vesicle"
}